positive regulation of maintenance of mitotic sister chromatid cohesion, centromeric [GO:2000720] (biological process) Also known as: positive regulation of maintenance of centromeric mitotic sister chromatin cohesion, positive regulation of maintenance of mitotic sister chromatin cohesion at centromere, positive regulation of maintenance of sister chromatin cohesion at centromere at mitosis Definition: Any process that activates or increases the frequency, rate or extent of maintenance of mitotic sister chromatid cohesion in the centromeric region. Relationships: is a type of positive regulation of maintenance of mitotic sister chromatid cohesion [GO:0034184]; is a type of regulation of maintenance of mitotic sister chromatid cohesion, centromeric [GO:2000718]; positively regulates GO:0071960 Sources: GOC:mah